{
  "term_label": "Unknown cellular component",
  "gene": "UniProtKB:Q5XLA6",
  "gene_symbol": "CARD17P",
  "gene_name": "Putative caspase recruitment domain-containing protein 17P",
  "term_id": "UNKNOWN:0003"
}